{
  "gene_symbol": "FABP12",
  "term_label": "fatty acid transport",
  "term_id": "GO:0015908",
  "gene_name": "Fatty acid-binding protein 12",
  "gene": "UniProtKB:A6NFH5"
}